{
  "term_label": "L-aspartate import across plasma membrane",
  "gene_symbol": "SLC1A3",
  "term_id": "GO:0140009",
  "gene": "UniProtKB:P43003",
  "gene_name": "Excitatory amino acid transporter 1"
}